peptide:proton symporter activity [GO:0015333] (molecular function) Relationships: is a type of solute:proton symporter activity [GO:0015295]; is a type of GO:1904680 Sources: GOC:mtg_transport, TC:2.A.17.-.- Also known as: peptide:hydrogen symporter activity Definition: Enables the transfer of a solute or solutes from one side of a membrane to the other according to the reaction: peptide(out) + H+(out) = peptide(in) + H+(in), up its concentration gradient. The transporter binds the solute and undergoes a series of conformational changes. Transport works equally well in either direction and is driven by hydrogen ion movement.